A2B adenosine receptor binding [GO:0031688] (molecular function) Definition: Binding to an A2B adenosine receptor. Also known as: A2B adenosine receptor ligand Relationships: is a type of adenosine receptor binding [GO:0031685] Sources: GOC:mah, GOC:nln